{
  "gene_symbol": "GCSAML",
  "term_label": "Unknown molecular function",
  "gene": "UniProtKB:Q5JQS6",
  "term_id": "UNKNOWN:0001",
  "gene_name": "Germinal center-associated signaling and motility-like protein"
}